negative regulation of neurogenesis [GO:0050768] (biological process) Sources: GOC:ai Relationships: is_a negative regulation of cell development [GO:0010721]; is a type of regulation of neurogenesis [GO:0050767]; is a type of negative regulation of nervous system development [GO:0051961]; negatively regulates GO:0022008 Definition: Any process that stops, prevents, or reduces the frequency, rate or extent of neurogenesis, the generation of cells within the nervous system. Also known as: down regulation of neurogenesis, down-regulation of neurogenesis, downregulation of neurogenesis, inhibition of neurogenesis Subtypes: negative regulation of neuroblast proliferation [GO:0007406], negative regulation of gliogenesis [GO:0014014], negative regulation of long-term neuronal synaptic plasticity [GO:0048171], negative regulation of short-term neuronal synaptic plasticity [GO:0048174], GO:0050771, negative regulation of dendrite morphogenesis [GO:0050774]